{
  "term_label": "Unknown molecular function",
  "term_id": "UNKNOWN:0001",
  "gene": "UniProtKB:Q5HY64",
  "gene_symbol": "FAM47C",
  "gene_name": "Putative protein FAM47C"
}